modification-dependent macromolecule catabolic process [GO:0043632] (biological process) Relationships: is a type of GO:0009057 Definition: The chemical reactions and pathways resulting in the breakdown of a macromolecule, initiated by covalent modification of the target molecule. Subtypes: modification-dependent protein catabolic process [GO:0019941], polyadenylation-dependent RNA catabolic process [GO:0043633], GO:1990074 Sources: GOC:jl